{
  "term_label": "Unknown cellular component",
  "gene": "UniProtKB:Q5TA78",
  "gene_name": "Late cornified envelope protein 4A",
  "term_id": "UNKNOWN:0003",
  "gene_symbol": "LCE4A"
}